{
  "gene_symbol": "CTXND2",
  "term_id": "UNKNOWN:0001",
  "gene_name": "Cortexin domain containing 2",
  "gene": "UniProtKB:A0A1B0GV90",
  "term_label": "Unknown molecular function"
}